negative regulation of non-canonical inflammasome complex assembly [GO:0160076] (biological process) Relationships: is a type of negative regulation of protein-containing complex assembly [GO:0031333]; is part of negative regulation of inflammasome-mediated signaling pathway [GO:0141086]; negatively regulates non-canonical inflammasome complex assembly [GO:0160075] Definition: Any process that stops, prevents or reduces the frequency, rate or extent of non-canonical inflammasome complex assembly. References: PMID:22002608, PMID:26375259